{
  "term_label": "spliceosomal complex",
  "gene_name": "ATP-dependent RNA helicase DHX15",
  "gene_symbol": "DHX15",
  "gene": "UniProtKB:O43143",
  "term_id": "GO:0005681"
}